{
  "gene_symbol": "HSF4",
  "gene": "UniProtKB:Q9ULV5",
  "term_label": "DNA-binding transcription factor activity",
  "term_id": "GO:0003700",
  "gene_name": "Heat shock factor protein 4"
}